{
  "gene_name": "Proline-rich protein 3",
  "gene": "UniProtKB:P79522",
  "term_label": "chromatin",
  "term_id": "GO:0000785",
  "gene_symbol": "PRR3"
}